{
  "term_label": "external side of plasma membrane",
  "term_id": "GO:0009897",
  "gene_symbol": "CLEC4C",
  "gene_name": "C-type lectin domain family 4 member C",
  "gene": "UniProtKB:Q8WTT0"
}